{
  "gene_symbol": "IGHV3-66",
  "gene": "UniProtKB:A0A0C4DH42",
  "gene_name": "Immunoglobulin heavy variable 3-66",
  "term_label": "Unknown cellular component",
  "term_id": "UNKNOWN:0003"
}